{
  "gene_symbol": "CENPV",
  "gene": "UniProtKB:Q7Z7K6",
  "term_id": "GO:0000776",
  "gene_name": "Centromere protein V",
  "term_label": "kinetochore"
}